{
  "gene_name": "Kelch-like protein 32",
  "term_label": "Cul3-RING ubiquitin ligase complex",
  "term_id": "GO:0031463",
  "gene": "UniProtKB:Q96NJ5",
  "gene_symbol": "KLHL32"
}